{
  "term_label": "rRNA (adenine-N6,N6-)-dimethyltransferase activity",
  "term_id": "GO:0000179",
  "gene": "UniProtKB:Q8WVM0",
  "gene_symbol": "TFB1M",
  "gene_name": "Dimethyladenosine transferase 1, mitochondrial"
}